{
  "gene_symbol": "TNFAIP3",
  "term_label": "protein deubiquitination involved in ubiquitin-dependent protein catabolic process",
  "term_id": "GO:0071947",
  "gene_name": "Tumor necrosis factor alpha-induced protein 3",
  "gene": "UniProtKB:P21580"
}